{
  "term_id": "GO:0005634",
  "gene": "UniProtKB:B7Z6K7",
  "gene_symbol": "ZNF814",
  "gene_name": "Zinc finger protein 814",
  "term_label": "nucleus"
}